{
  "gene": "UniProtKB:Q03721",
  "term_label": "action potential",
  "gene_symbol": "KCNC4",
  "term_id": "GO:0001508",
  "gene_name": "Potassium voltage-gated channel subfamily C member 4"
}